{
  "gene": "UniProtKB:P20742",
  "gene_name": "Pregnancy zone protein",
  "term_label": "Unknown biological process",
  "gene_symbol": "PZP",
  "term_id": "UNKNOWN:0002"
}